{
  "gene_name": "Circadian locomoter output cycles protein kaput",
  "gene_symbol": "CLOCK",
  "gene": "UniProtKB:O15516",
  "term_label": "regulation of transcription by RNA polymerase II",
  "term_id": "GO:0006357"
}